ascospore formation [GO:0030437] (biological process) Definition: The process in which cells that are products of meiosis acquire the specialized features of ascospores. Ascospores are generally found in clusters of four or eight spores within a single mother cell, the ascus, and are characteristic of the ascomycete fungi (phylum Ascomycota). Relationships: is a type of reproductive process in single-celled organism [GO:0022413]; is_a GO:0043935; is a type of cell development [GO:0048468]; is a type of meiotic cell cycle process [GO:1903046] Regulation: regulated by regulation of ascospore formation [GO:0034307]; RO_0002213 by positive regulation of ascospore formation [GO:0075296]; negatively regulated by negative regulation of ascospore formation [GO:0075297] Note: Note that ascospores and asci are separate biological structures. The ascus is the structure that contain the ascospores, but the development of the ascus is a different process than the formation of the ascospores themselves; for instance, some mutations affect sporulation without affecting ascus development. For this reason, GO:0030437 ascospore formation and GO:0075317 ascus development are different terms and are not linked. References: PMID:16339736 Sources: GOC:di, GOC:mah, GOC:mcc Also known as: spore formation, sporulation, ascospore biosynthesis